vesicle budding from membrane [GO:0006900] (biological process) Subtypes: COPI-coated vesicle budding [GO:0035964], GO:0048194, synaptic vesicle budding [GO:0070142], intralumenal vesicle formation [GO:0070676], COPII-coated vesicle budding [GO:0090114] Sources: GOC:jid, GOC:tb Definition: The evagination of a membrane, resulting in formation of a vesicle. Also known as: membrane evagination, vesicle biosynthesis, vesicle formation, nonselective vesicle assembly, single organism membrane budding, single-organism membrane budding, vesicle budding Relationships: is a type of vesicle organization [GO:0016050]; is a type of membrane organization [GO:0061024]; is part of vesicle-mediated transport [GO:0016192]